protein-N(PI)-phosphohistidine-mannitol phosphotransferase system transmembrane transporter activity [GO:0022872] (molecular function) Sources: GOC:mtg_transport, ISBN:0815340729 Also known as: mannitol PTS transporter activity Definition: Catalysis of the PEP-dependent, phosphoryl transfer-driven transport of substances across a membrane. The transport happens by catalysis of the reaction: protein N-phosphohistidine + mannitol(out) = protein histidine + mannitol phosphate(in). This differs from primary and secondary active transport in that the solute is modified during transport. Relationships: is a type of protein-N(PI)-phosphohistidine-sugar phosphotransferase activity [GO:0008982]; is a type of mannitol transmembrane transporter activity [GO:0015575]